{
  "term_label": "extracellular space",
  "term_id": "GO:0005615",
  "gene_name": "Adenosine deaminase 2",
  "gene": "UniProtKB:Q9NZK5",
  "gene_symbol": "ADA2"
}